{
  "term_label": "ubiquitin protein ligase activity",
  "gene_symbol": "TRIM61",
  "gene_name": "Putative tripartite motif-containing protein 61",
  "gene": "UniProtKB:Q5EBN2",
  "term_id": "GO:0061630"
}